{
  "gene": "UniProtKB:O75367",
  "gene_symbol": "MACROH2A1",
  "term_label": "negative regulation of transcription of nucleolar large rRNA by RNA polymerase I",
  "gene_name": "Core histone macro-H2A.1",
  "term_id": "GO:1901837"
}